{
  "gene": "UniProtKB:P48551",
  "term_id": "GO:0004905",
  "gene_symbol": "IFNAR2",
  "gene_name": "Interferon alpha_beta receptor 2",
  "term_label": "type I interferon receptor activity"
}